{
  "gene": "UniProtKB:Q5VTY9",
  "gene_name": "Protein-cysteine N-palmitoyltransferase HHAT",
  "gene_symbol": "HHAT",
  "term_label": "Unknown biological process",
  "term_id": "UNKNOWN:0002"
}